{
  "gene_name": "26S proteasome regulatory subunit 10B",
  "term_id": "GO:0036402",
  "term_label": "proteasome-activating activity",
  "gene": "UniProtKB:P62333",
  "gene_symbol": "PSMC6"
}